{
  "gene": "UniProtKB:Q9UMX9",
  "term_label": "sucrose:proton symporter activity",
  "term_id": "GO:0008506",
  "gene_name": "Membrane-associated transporter protein",
  "gene_symbol": "SLC45A2"
}